{
  "gene_symbol": "IGF2BP1",
  "gene_name": "Insulin-like growth factor 2 mRNA-binding protein 1",
  "term_label": "nervous system development",
  "term_id": "GO:0007399",
  "gene": "UniProtKB:Q9NZI8"
}